{
  "term_label": "xanthine dehydrogenase activity",
  "gene": "UniProtKB:P47989",
  "gene_symbol": "XDH",
  "gene_name": "Xanthine dehydrogenase_oxidase",
  "term_id": "GO:0004854"
}